{
  "term_label": "(3S)-3-hydroxyacyl-CoA dehydrogenase (NAD+) activity",
  "gene_name": "Peroxisomal bifunctional enzyme",
  "gene": "UniProtKB:Q08426",
  "gene_symbol": "EHHADH",
  "term_id": "GO:0003857"
}